positive regulation of cellular response to X-ray [GO:2000685] (biological process) Relationships: is a type of positive regulation of cellular process [GO:0048522]; is a type of positive regulation of response to stimulus [GO:0048584]; is a type of GO:2000683; positively regulates cellular response to X-ray [GO:0071481] Sources: GOC:obol Also known as: positive regulation of cellular response to X-ray radiation stimulus Definition: Any process that activates or increases the frequency, rate or extent of cellular response to X-ray.